{
  "term_label": "phospholipase C-activating G protein-coupled receptor signaling pathway",
  "term_id": "GO:0007200",
  "gene": "UniProtKB:P32239",
  "gene_name": "Gastrin_cholecystokinin type B receptor",
  "gene_symbol": "CCKBR"
}